{
  "gene_name": "HHIP-like protein 1",
  "gene": "UniProtKB:Q96JK4",
  "term_label": "Unknown biological process",
  "gene_symbol": "HHIPL1",
  "term_id": "UNKNOWN:0002"
}